{
  "gene": "UniProtKB:Q96EY1",
  "gene_symbol": "DNAJA3",
  "term_label": "mitochondrion organization",
  "term_id": "GO:0007005",
  "gene_name": "DnaJ homolog subfamily A member 3, mitochondrial"
}